symbiont entry into host cell [GO:0046718] (biological process) Also known as: entry of virus into host cell, phage translocation, viral entry into host cell, viral penetration, virion penetration, virion penetration into host cell, virus entry into host cell Definition: The process by which a symbiont breaches the plasma membrane or cell envelope and enters the host cell. The process ends when the symbiont or its genome is released into the host cell. Sources: GOC:jl Subtypes: endocytosis involved in viral entry into host cell [GO:0075509], GO:0085017 Relationships: is_a GO:0044409; is part of viral life cycle [GO:0019058] Regulation: regulated by regulation of viral entry into host cell [GO:0046596]; positively regulated by positive regulation of viral entry into host cell [GO:0046598]; RO_0002212 by negative regulation of fusion of virus membrane with host plasma membrane [GO:1903914] Note: Viral attachment to the host cell is not part of viral entry in GO because virus attachment does not always lead to viral entry: attachment can also result in the virion being carried by the host cell to another location.